L-lysine 6-oxidase activity [GO:0033736] (molecular function) Relationships: is a type of L-amino-acid oxidase activity [GO:0001716] Also known as: L-lysine-epsilon-oxidase activity, L-lysine:oxygen 6-oxidoreductase (deaminating) activity, Lod, LodA, marinocine Sources: RHEA:22548 Definition: Catalysis of the reaction: H2O + L-lysine + O2 = (S)-2-amino-6-oxohexanoate + H2O2 + NH4+.